{
  "term_label": "DNA-binding transcription factor activity, RNA polymerase II-specific",
  "term_id": "GO:0000981",
  "gene": "UniProtKB:Q12857",
  "gene_name": "Nuclear factor 1 A-type",
  "gene_symbol": "NFIA"
}